{
  "gene_symbol": "DCLK1",
  "term_id": "GO:0048675",
  "term_label": "axon extension",
  "gene": "UniProtKB:O15075",
  "gene_name": "Serine_threonine-protein kinase DCLK1"
}